{
  "gene_name": "E3 ubiquitin-protein ligase SIAH2",
  "gene_symbol": "SIAH2",
  "gene": "UniProtKB:O43255",
  "term_label": "proteasome-mediated ubiquitin-dependent protein catabolic process",
  "term_id": "GO:0043161"
}